{
  "gene": "UniProtKB:Q9ULH1",
  "gene_name": "Arf-GAP with SH3 domain, ANK repeat and PH domain-containing protein 1",
  "term_id": "GO:0060271",
  "gene_symbol": "ASAP1",
  "term_label": "cilium assembly"
}